{
  "term_label": "extracellular space",
  "gene_name": "Leucine-rich repeat transmembrane protein FLRT3",
  "gene_symbol": "FLRT3",
  "term_id": "GO:0005615",
  "gene": "UniProtKB:Q9NZU0"
}